{
  "gene": "UniProtKB:Q5EG05",
  "term_label": "Unknown molecular function",
  "gene_name": "Caspase recruitment domain-containing protein 16",
  "term_id": "UNKNOWN:0001",
  "gene_symbol": "CARD16"
}